steroid 22S-hydroxylase activity [GO:0160191] (molecular function) Definition: Catalysis of the reaction: a C28-steroid + O2 + reduced NADPH--hemoprotein reductase = a (22S)-22-hydroxy C28-steroid + H+ + H2O + oxidized NADPH--hemoprotein reductase. Also catalyzes the C-22 hydroxylation of a variety of C27 and C29 steroids. Sources: EC:1.14.14.178 Also known as: steroid C-22 hydroxylase activity Relationships: is a type of steroid hydroxylase activity [GO:0008395]; is_a oxidoreductase activity, acting on paired donors, with incorporation or reduction of molecular oxygen, reduced flavin or flavoprotein as one donor, and incorporation of one atom of oxygen [GO:0016712]